CDP phosphatase activity [GO:0036384] (molecular function) Sources: GOC:al, RHEA:64880 Definition: Catalysis of the reaction: CDP + H2O = CMP + phosphate. Relationships: is a type of nucleoside diphosphate phosphatase activity [GO:0017110] Also known as: CDP diphosphatase activity, CDPase activity, cytidine diphosphatase activity, cytidine-diphosphatase activity